{
  "gene_symbol": "OST4",
  "gene": "UniProtKB:P0C6T2",
  "term_id": "GO:0018279",
  "gene_name": "Dolichyl-diphosphooligosaccharide--protein glycosyltransferase subunit 4",
  "term_label": "protein N-linked glycosylation via asparagine"
}